{
  "gene": "UniProtKB:P61266",
  "term_label": "presynaptic active zone membrane",
  "gene_symbol": "STX1B",
  "gene_name": "Syntaxin-1B",
  "term_id": "GO:0048787"
}